{
  "gene_name": "Zinc finger protein 83",
  "term_id": "UNKNOWN:0003",
  "gene_symbol": "ZNF83",
  "gene": "UniProtKB:P51522",
  "term_label": "Unknown cellular component"
}